{
  "term_id": "GO:0008180",
  "term_label": "COP9 signalosome",
  "gene": "UniProtKB:Q92905",
  "gene_symbol": "COPS5",
  "gene_name": "COP9 signalosome complex subunit 5"
}